{
  "term_id": "GO:0005886",
  "gene_symbol": "GRAMD1B",
  "gene_name": "Protein Aster-B",
  "gene": "UniProtKB:Q3KR37",
  "term_label": "plasma membrane"
}